ER body [GO:0010168] (cellular component) Definition: A novel compartment found in plant cells that is derived from the ER. The structures have a characteristic shape and size (10 mm long and 0.5 mm wide) and are surrounded with ribosomes. They have been found in Arabidopsis thaliana and related Brassicaceae species. References: PMID:11577182 Also known as: endoplasmic reticulum body Relationships: is a type of intracellular membrane-bounded organelle [GO:0043231]